{
  "gene_name": "Nuclear factor 1 X-type",
  "gene_symbol": "NFIX",
  "term_label": "RNA polymerase II cis-regulatory region sequence-specific DNA binding",
  "term_id": "GO:0000978",
  "gene": "UniProtKB:Q14938"
}